{
  "gene_name": "Endogenous retrovirus group K member 10 Pol protein",
  "term_label": "Unknown biological process",
  "gene": "UniProtKB:P10266",
  "term_id": "UNKNOWN:0002",
  "gene_symbol": "ERVK-10"
}